{
  "term_label": "microtubule cytoskeleton organization",
  "gene_symbol": "TUBA3C",
  "gene": "UniProtKB:P0DPH7",
  "term_id": "GO:0000226",
  "gene_name": "Tubulin alpha-3C chain"
}